{
  "term_label": "Golgi apparatus",
  "gene": "UniProtKB:Q7RTS9",
  "gene_symbol": "DYM",
  "gene_name": "Dymeclin",
  "term_id": "GO:0005794"
}